{
  "gene_symbol": "IGHV3-7",
  "term_label": "antigen binding",
  "term_id": "GO:0003823",
  "gene_name": "Immunoglobulin heavy variable 3-7",
  "gene": "UniProtKB:P01780"
}